{
  "gene": "UniProtKB:A0A5F9ZGZ6",
  "term_id": "UNKNOWN:0002",
  "gene_symbol": "A0A5F9ZGZ6",
  "gene_name": "Rho guanine nucleotide exchange factor 5_35 N-terminal domain-containing protein",
  "term_label": "Unknown biological process"
}